16-hydroxysteroid epimerase activity [GO:0047524] (molecular function) Relationships: is a type of GO:0016854 Also known as: 16-hydroxysteroid 16-epimerase activity Definition: Catalysis of the reaction: 16-alpha-hydroxysteroid = 16-beta-hydroxysteroid. Sources: RHEA:15829